{
  "term_label": "cell surface receptor signaling pathway",
  "gene_name": "T cell receptor beta variable 6-6",
  "gene_symbol": "TRBV6-6",
  "term_id": "GO:0007166",
  "gene": "UniProtKB:A0A0A6YYG2"
}